{
  "gene": "UniProtKB:Q9HC07",
  "term_id": "GO:0032468",
  "gene_name": "Transmembrane protein 165",
  "gene_symbol": "TMEM165",
  "term_label": "Golgi calcium ion homeostasis"
}